sulfite reductase (coenzyme F420) activity [GO:0052806] (molecular function) Also known as: coenzyme F420-dependent sulfite reductase activity, coenzyme F420-sulfite reductase activity, hydrogen-sulfide:coenzyme F420 oxidoreductase activity, sulfite:reduced coenzyme F420 reductase activity Relationships: is a type of oxidoreductase activity, acting on a sulfur group of donors [GO:0016667] Definition: Catalysis of the reaction: sulfite + 3 1,5-dihydrocoenzyme F420 = hydrogen sulfide + 3 H2O + 3 coenzyme F420. 1,5-dihydrocoenzyme F420 is also known as reduced coenzyme F420. References: PMID:16048999 Sources: GOC:mengo_curators